{
  "term_id": "GO:0048663",
  "gene_name": "Elongin BC and Polycomb repressive complex 2-associated protein",
  "term_label": "neuron fate commitment",
  "gene_symbol": "EPOP",
  "gene": "UniProtKB:A6NHQ4"
}